{
  "term_label": "endonucleolytic cleavage to generate mature 5'-end of SSU-rRNA from (SSU-rRNA, 5.8S rRNA, LSU-rRNA)",
  "gene_symbol": "NOP9",
  "term_id": "GO:0000472",
  "gene": "UniProtKB:Q86U38",
  "gene_name": "Nucleolar protein 9"
}